{
  "term_label": "G protein-coupled receptor activity",
  "gene_symbol": "ADGRG4",
  "term_id": "GO:0004930",
  "gene_name": "Adhesion G-protein coupled receptor G4",
  "gene": "UniProtKB:Q8IZF6"
}